{
  "gene_symbol": "SMR3B",
  "gene_name": "Submaxillary gland androgen-regulated protein 3B",
  "term_label": "regulation of sensory perception of pain",
  "term_id": "GO:0051930",
  "gene": "UniProtKB:P02814"
}